{
  "gene_symbol": "FHL3",
  "term_label": "stress fiber",
  "term_id": "GO:0001725",
  "gene": "UniProtKB:Q13643",
  "gene_name": "Four and a half LIM domains protein 3"
}